{
  "gene_symbol": "IGHV1-69D",
  "gene_name": "Immunoglobulin heavy variable 1-69D",
  "term_id": "GO:0003823",
  "gene": "UniProtKB:A0A0B4J2H0",
  "term_label": "antigen binding"
}